macromolecular conformation isomerase activity [GO:0120543] (molecular function) Sources: EC:5.6.-.- Relationships: is_a isomerase activity [GO:0016853] Definition: Catalysis of a reaction that alters the macromolecular conformation of a molecule. Subtypes: polypeptide conformation or assembly isomerase activity [GO:0120544], nucleic acid conformation isomerase activity [GO:0120545]